{
  "term_id": "GO:0032456",
  "gene_symbol": "RAB8B",
  "term_label": "endocytic recycling",
  "gene": "UniProtKB:Q92930",
  "gene_name": "Ras-related protein Rab-8B"
}